{
  "term_label": "chemorepellent activity",
  "gene_name": "Semaphorin-3E",
  "gene_symbol": "SEMA3E",
  "term_id": "GO:0045499",
  "gene": "UniProtKB:O15041"
}